cell projection organization [GO:0030030] (biological process) Relationships: is a type of cellular component organization [GO:0016043] Definition: A process that is carried out at the cellular level which results in the assembly, arrangement of constituent parts, or disassembly of a prolongation or process extending from a cell, e.g. a flagellum or axon. References: PMID:16318917 Sources: GOC:jl, GOC:mah Regulation: RO_0002211 by regulation of cell projection organization [GO:0031344]; RO_0002212 by negative regulation of cell projection organization [GO:0031345]; positively regulated by GO:0031346 Also known as: cell projection organisation, cell projection organization and biogenesis, cell surface structure organization and biogenesis Subtypes: cell projection assembly [GO:0030031], pilus organization [GO:0043711], bacterial-type flagellum organization [GO:0044781], cell projection morphogenesis [GO:0048858], plasma membrane bounded cell projection organization [GO:0120036]